{
  "term_id": "GO:0005634",
  "gene_name": "NK1 transcription factor-related protein 2",
  "term_label": "nucleus",
  "gene": "UniProtKB:Q9UD57",
  "gene_symbol": "NKX1-2"
}